mannosyl-diinositol phosphorylceramide phospholipase activity [GO:0052715] (MF) Definition: Catalysis of the reaction: mannosyl-diinositol phosphorylceramide + H2O = C26-phytoceramide + mannosyldiphosphorylinositol. Relationships: is a type of inositol phosphorylceramide phospholipase activity [GO:0052713] Sources: GOC:ai